{
  "gene_symbol": "COL4A3",
  "term_label": "extracellular matrix",
  "gene_name": "Collagen alpha-3(IV) chain",
  "gene": "UniProtKB:Q01955",
  "term_id": "GO:0031012"
}